{
  "term_label": "endoplasmic reticulum membrane",
  "term_id": "GO:0005789",
  "gene_name": "Transmembrane protein 258",
  "gene": "UniProtKB:P61165",
  "gene_symbol": "TMEM258"
}